{
  "term_label": "Unknown cellular component",
  "term_id": "UNKNOWN:0003",
  "gene": "UniProtKB:A6NFU0",
  "gene_name": "Ig-like V-type domain-containing protein FAM187A",
  "gene_symbol": "FAM187A"
}